{
  "gene_name": "Protein S100-B",
  "term_id": "GO:0043123",
  "gene": "UniProtKB:P04271",
  "term_label": "positive regulation of canonical NF-kappaB signal transduction",
  "gene_symbol": "S100B"
}